positive regulation of prostaglandin biosynthetic process [GO:0031394] (biological process) Subtypes: positive regulation of fever generation by positive regulation of prostaglandin biosynthesis [GO:0071811] Definition: Any process that activates or increases the frequency, rate or extent of the chemical reactions and pathways resulting in the formation of prostaglandin. Also known as: positive regulation of prostaglandin anabolism, positive regulation of prostaglandin biosynthesis, positive regulation of prostaglandin formation, positive regulation of prostaglandin synthesis, up regulation of prostaglandin biosynthetic process, up-regulation of prostaglandin biosynthetic process, upregulation of prostaglandin biosynthetic process, activation of prostaglandin biosynthetic process, stimulation of prostaglandin biosynthetic process Sources: GOC:mah Relationships: is a type of regulation of prostaglandin biosynthetic process [GO:0031392]; is a type of positive regulation of unsaturated fatty acid biosynthetic process [GO:2001280]; RO_0002213 prostaglandin biosynthetic process [GO:0001516]